{
  "gene_name": "OTU domain-containing protein 1",
  "term_label": "Unknown biological process",
  "term_id": "UNKNOWN:0002",
  "gene_symbol": "OTUD1",
  "gene": "UniProtKB:Q5VV17"
}